{
  "gene": "UniProtKB:O00512",
  "term_id": "GO:0045944",
  "gene_name": "B-cell CLL_lymphoma 9 protein",
  "gene_symbol": "BCL9",
  "term_label": "positive regulation of transcription by RNA polymerase II"
}